regulation of mast cell proliferation [GO:0070666] (biological process) Relationships: is a type of regulation of leukocyte proliferation [GO:0070663]; regulates mast cell proliferation [GO:0070662] Subtypes: GO:0070667, positive regulation of mast cell proliferation [GO:0070668] Sources: GOC:add, GOC:mah Definition: Any process that modulates the frequency, rate or extent of mast cell proliferation.